{
  "gene": "UniProtKB:P41439",
  "term_label": "cell adhesion",
  "gene_name": "Folate receptor gamma",
  "gene_symbol": "FOLR3",
  "term_id": "GO:0007155"
}